{
  "gene": "UniProtKB:Q9HAU0",
  "gene_symbol": "PLEKHA5",
  "term_label": "phosphatidylinositol-5-phosphate binding",
  "term_id": "GO:0010314",
  "gene_name": "Pleckstrin homology domain-containing family A member 5"
}